{
  "gene_symbol": "CDH9",
  "term_label": "catenin complex",
  "gene": "UniProtKB:Q9ULB4",
  "gene_name": "Cadherin-9",
  "term_id": "GO:0016342"
}